{
  "term_id": "GO:0005737",
  "gene_name": "Tumor protein D54",
  "term_label": "cytoplasm",
  "gene": "UniProtKB:O43399",
  "gene_symbol": "TPD52L2"
}